{
  "term_id": "GO:0003682",
  "gene_symbol": "STAG3",
  "gene": "UniProtKB:Q9UJ98",
  "gene_name": "Cohesin subunit SA-3",
  "term_label": "chromatin binding"
}